{
  "term_label": "regulation of apoptotic process",
  "gene": "UniProtKB:Q9P275",
  "gene_name": "Ubiquitin carboxyl-terminal hydrolase 36",
  "term_id": "GO:0042981",
  "gene_symbol": "USP36"
}